{
  "term_label": "Unknown biological process",
  "gene_name": "Speedy protein E12",
  "gene": "UniProtKB:P0DUX1",
  "term_id": "UNKNOWN:0002",
  "gene_symbol": "SPDYE12"
}